{
  "gene_name": "Integrin beta-1-binding protein 1",
  "gene_symbol": "ITGB1BP1",
  "term_label": "ruffle",
  "gene": "UniProtKB:O14713",
  "term_id": "GO:0001726"
}